{
  "gene_name": "Fas apoptotic inhibitory molecule 1",
  "term_id": "UNKNOWN:0003",
  "term_label": "Unknown cellular component",
  "gene_symbol": "FAIM",
  "gene": "UniProtKB:Q9NVQ4"
}